positive regulation of optic nerve formation [GO:2000597] (biological process) Sources: GOC:obol Definition: Any process that activates or increases the frequency, rate or extent of optic nerve formation. Also known as: positive regulation of CN II biosynthesis, positive regulation of CN II formation Relationships: is a type of GO:0051094; is a type of regulation of optic nerve formation [GO:2000595]; positively regulates GO:0021634